2-dehydropantoate 2-reductase activity [GO:0008677] (molecular function) Definition: Catalysis of the reaction: (R)-pantoate + NADP+ = 2-dehydropantoate + H+ + NADPH. Also known as: (R)-pantoate:NADP+ 2-oxidoreductase activity, 2-ketopantoate reductase activity, 2-ketopantoic acid reductase activity, 2-oxopantoate reductase activity, KPA reductase activity, ketopantoate reductase activity, ketopantoic acid reductase activity Relationships: is a type of oxidoreductase activity, acting on the CH-OH group of donors, NAD or NADP as acceptor [GO:0016616] Sources: EC:1.1.1.169, RHEA:16233